{
  "term_label": "melanosome membrane",
  "gene_symbol": "GPR143",
  "gene": "UniProtKB:P51810",
  "term_id": "GO:0033162",
  "gene_name": "G-protein coupled receptor 143"
}